{
  "term_label": "synapse",
  "gene_symbol": "HTR3D",
  "gene_name": "5-hydroxytryptamine receptor 3D",
  "gene": "UniProtKB:Q70Z44",
  "term_id": "GO:0045202"
}